{
  "term_label": "Unknown biological process",
  "gene": "UniProtKB:Q96BQ5",
  "gene_name": "Coiled-coil domain-containing protein 127",
  "term_id": "UNKNOWN:0002",
  "gene_symbol": "CCDC127"
}